{
  "term_label": "plasma membrane",
  "gene_name": "Matrix metalloproteinase-14",
  "gene": "UniProtKB:P50281",
  "gene_symbol": "MMP14",
  "term_id": "GO:0005886"
}